{
  "term_id": "GO:0035336",
  "term_label": "long-chain fatty-acyl-CoA metabolic process",
  "gene_name": "Long-chain-fatty-acid--CoA ligase 4",
  "gene_symbol": "ACSL4",
  "gene": "UniProtKB:O60488"
}